{
  "term_id": "GO:0000978",
  "gene_symbol": "PAX1",
  "gene": "UniProtKB:P15863",
  "term_label": "RNA polymerase II cis-regulatory region sequence-specific DNA binding",
  "gene_name": "Paired box protein Pax-1"
}